{
  "term_id": "GO:0006457",
  "gene_symbol": "CLGN",
  "term_label": "protein folding",
  "gene": "UniProtKB:O14967",
  "gene_name": "Calmegin"
}